{
  "gene_name": "Small kinetochore-associated protein",
  "term_id": "GO:0051988",
  "term_label": "regulation of attachment of spindle microtubules to kinetochore",
  "gene_symbol": "KNSTRN",
  "gene": "UniProtKB:Q9Y448"
}